{
  "term_id": "GO:0001227",
  "gene_symbol": "KRBOX4",
  "gene": "UniProtKB:Q5JUW0",
  "gene_name": "KRAB domain-containing protein 4",
  "term_label": "DNA-binding transcription repressor activity, RNA polymerase II-specific"
}